positive regulation of diorcinol biosynthetic process [GO:1900657] (biological process) Definition: Any process that activates or increases the frequency, rate or extent of diorcinol biosynthetic process. Relationships: is_a GO:1900378; is a type of GO:1900655; positively regulates diorcinol biosynthetic process [GO:1900572] Also known as: activation of diorcinol anabolism, activation of diorcinol biosynthesis, activation of diorcinol formation, activation of diorcinol synthesis, positive regulation of diorcinol anabolism, positive regulation of diorcinol biosynthesis, positive regulation of diorcinol formation, positive regulation of diorcinol synthesis, up regulation of diorcinol anabolism, up regulation of diorcinol biosynthesis, up regulation of diorcinol biosynthetic process, up regulation of diorcinol formation, up regulation of diorcinol synthesis, up-regulation of diorcinol anabolism, up-regulation of diorcinol biosynthesis, up-regulation of diorcinol biosynthetic process, up-regulation of diorcinol formation, up-regulation of diorcinol synthesis, upregulation of diorcinol anabolism, upregulation of diorcinol biosynthesis, upregulation of diorcinol biosynthetic process, upregulation of diorcinol formation, upregulation of diorcinol synthesis, activation of diorcinol biosynthetic process Sources: GOC:TermGenie, GOC:di